positive regulation of adenylate cyclase activity [GO:0045762] (biological process) Sources: GOC:go_curators Relationships: is a type of positive regulation of cyclase activity [GO:0031281]; is a type of regulation of adenylate cyclase activity [GO:0045761]; is a type of positive regulation of lyase activity [GO:0051349]; positively regulates GO:0004016 Definition: Any process that activates or increases the frequency, rate or extent of adenylate cyclase activity. Also known as: positive regulation of adenylyl cyclase activity, up regulation of adenylate cyclase activity, up-regulation of adenylate cyclase activity, upregulation of adenylate cyclase activity, stimulation of adenylate cyclase activity, adenylate cyclase activator Subtypes: activation of adenylate cyclase activity [GO:0007190]